{
  "gene": "UniProtKB:Q96GA7",
  "term_label": "L-serine ammonia-lyase activity",
  "term_id": "GO:0003941",
  "gene_symbol": "SDSL",
  "gene_name": "Serine dehydratase-like"
}